{
  "gene": "UniProtKB:P07942",
  "gene_name": "Laminin subunit beta-1",
  "gene_symbol": "LAMB1",
  "term_id": "GO:0005201",
  "term_label": "extracellular matrix structural constituent"
}